{
  "gene_symbol": "PELI2",
  "gene": "UniProtKB:Q9HAT8",
  "term_id": "UNKNOWN:0003",
  "gene_name": "E3 ubiquitin-protein ligase pellino homolog 2",
  "term_label": "Unknown cellular component"
}